indoxyl-UDPG glucosyltransferase activity [GO:0050507] (molecular function) Definition: Catalysis of the reaction: indoxyl + UDP-D-glucose = H+ + indican + UDP. Sources: EC:2.4.1.220, RHEA:12004 Also known as: UDP-glucose:indoxyl 3-O-beta-D-glucosyltransferase activity, indoxyl-UDPG-glucosyltransferase activity Relationships: is a type of UDP-glucosyltransferase activity [GO:0035251]